{
  "gene": "UniProtKB:O43809",
  "term_label": "mRNA 3'-UTR AU-rich region binding",
  "gene_name": "Cleavage and polyadenylation specificity factor subunit 5",
  "gene_symbol": "NUDT21",
  "term_id": "GO:0035925"
}